(Z)-nonadeca-1,14-diene metabolic process [GO:1900878] (biological process) Definition: The chemical reactions and pathways involving (Z)-nonadeca-1,14-diene. Relationships: is a type of olefin metabolic process [GO:1900673] Subtypes: (Z)-nonadeca-1,14-diene biosynthetic process [GO:1900879] Also known as: (Z)-nonadeca-1,14-diene metabolism Sources: GOC:TermGenie, GOC:mengo_curators